{
  "gene": "UniProtKB:Q15025",
  "term_label": "Unknown cellular component",
  "term_id": "UNKNOWN:0003",
  "gene_symbol": "TNIP1",
  "gene_name": "TNFAIP3-interacting protein 1"
}